{
  "term_id": "GO:0008017",
  "gene_name": "Cilia- and flagella-associated protein 157",
  "gene_symbol": "CFAP157",
  "term_label": "microtubule binding",
  "gene": "UniProtKB:Q5JU67"
}